{
  "term_label": "intracellularly calcium-gated chloride channel activity",
  "gene_symbol": "ANO1",
  "gene": "UniProtKB:Q5XXA6",
  "term_id": "GO:0005229",
  "gene_name": "Anoctamin-1"
}